nucleotide-excision repair [GO:0006289] (BP) Note: Note that although intrastrand cross-link repair is not exactly synonymous with nucleotide excision repair, nucleotide excision repair includes the repair of intrastrand cross-links. The synonym field is being used to reflect the broad substrate specificity of nucleotide excision repair. Relationships: is_a DNA repair [GO:0006281] Regulation: RO_0002211 by regulation of nucleotide-excision repair [GO:2000819] Also known as: NER, pyrimidine-dimer repair, DNA damage excision, intrastrand cross-link repair Definition: A DNA repair process in which a small region of the strand surrounding the damage is removed from the DNA helix as an oligonucleotide. The small gap left in the DNA helix is filled in by the sequential action of DNA polymerase and DNA ligase. Nucleotide excision repair recognizes a wide range of substrates, including damage caused by UV irradiation (pyrimidine dimers and 6-4 photoproducts) and chemicals (intrastrand cross-links and bulky adducts). Subtypes: GO:0000720, transcription-coupled nucleotide-excision repair [GO:0006283], global genome nucleotide-excision repair [GO:0070911], nucleotide-excision repair involved in interstrand cross-link repair [GO:1901255] References: PMID:10197977